beta-carotene 3-hydroxylase activity [GO:0010291] (molecular function) References: PMID:16492736 Sources: RHEA:30331 Definition: Catalysis of the reaction: all-trans-beta-carotene + 4 H+ + 2 O2 + 4 reduced [2Fe-2S]-[ferredoxin] = all-trans-zeaxanthin + 2 H2O + 4 oxidized [2Fe-2S]-[ferredoxin]. Also known as: beta-carotene hydroxylase activity, carotene beta-ring hydroxylase activity Relationships: is a type of monooxygenase activity [GO:0004497]